{
  "term_label": "plasma membrane",
  "gene": "UniProtKB:Q9C0C4",
  "gene_symbol": "SEMA4C",
  "term_id": "GO:0005886",
  "gene_name": "Semaphorin-4C"
}